cell-substrate junction assembly [GO:0007044] (biological process) Relationships: is a type of cell junction assembly [GO:0034329]; is a type of cell-substrate junction organization [GO:0150115] Sources: GOC:mah Subtypes: hemidesmosome assembly [GO:0031581], focal adhesion assembly [GO:0048041] Note: The primary label for merged term was 'cell-substrate adherens junction assembly' GO:0007045. The term was merged into the parent 'cell-substrate junction assembly', because, based on the most recent litarature, 'adherens junction' is always a 'cell-cell junction' (PMID:20571587, PMID:17854762, PMID:21422226, PMID:28096264, PMID:28401269, PMID:26923917). Definition: The aggregation, arrangement and bonding together of a set of components to form a junction between a cell and its substrate. Also known as: cell-substrate adherens junction assembly Regulation: regulated by regulation of cell-substrate junction assembly [GO:0090109]